histone H3K4me/H3K4me2/H3K4me3 demethylase activity [GO:0034647] (molecular function) Also known as: histone H3-K4me2 demethylase activity, histone H3K4me2 demethylase activity, histone H3-tri/di/monomethyl-lysine-4 demethylase activity, histone demethylase activity (H3-K4-me3 specific), histone demethylase activity (H3-trimethyl-K4 specific), H3K4me3 demethylase activity, histone H3-K4me3 demethylase activity Relationships: is_a 2-oxoglutarate-dependent dioxygenase activity [GO:0016706]; is a type of histone H3K4 demethylase activity [GO:0032453] References: PMID:17550896, PMID:22473470 Note: Comment: Note that the residue position corresponds to the canonical human H3 histone (UniProtKB:P84243); this residue is conserved across all eukaryotes. Residue 1 is the first residue following removal of the initiating Methionine (Met). Note that each histone is encoded by multiple genes, and sequences may vary across different genes within an organism. Definition: Catalysis of the removal of a methyl group from a tri, a di or a monomethyl-lysine residue at position 4 of the histone H3 protein. This is a dioxygenase reaction that is dependent on Fe(II) and 2-oxoglutarate.